{
  "term_label": "morphogenesis of an epithelium",
  "gene": "UniProtKB:P35900",
  "gene_symbol": "KRT20",
  "term_id": "GO:0002009",
  "gene_name": "Keratin, type I cytoskeletal 20"
}